protein homooligomerization [GO:0051260] (biological process) Regulation: regulated by regulation of protein homooligomerization [GO:0032462]; negatively regulated by negative regulation of protein homooligomerization [GO:0032463]; RO_0002213 by GO:0032464 Subtypes: GO:0051289, GO:0070207 Also known as: protein homooligomer assembly, protein homooligomer biosynthesis, protein homooligomer biosynthetic process, protein homooligomer formation, protein homooligomerization activity Definition: The process of creating protein oligomers, compounds composed of a small number, usually between three and ten, of identical component monomers. Oligomers may be formed by the polymerization of a number of monomers or the depolymerization of a large protein polymer. Relationships: is a type of GO:0051259 Sources: GOC:ai